{
  "term_id": "UNKNOWN:0001",
  "gene": "UniProtKB:Q6UWN5",
  "gene_symbol": "LYPD5",
  "term_label": "Unknown molecular function",
  "gene_name": "Ly6_PLAUR domain-containing protein 5"
}